{
  "term_label": "nucleus",
  "gene_symbol": "CUX2",
  "term_id": "GO:0005634",
  "gene": "UniProtKB:O14529",
  "gene_name": "Homeobox protein cut-like 2"
}